{
  "term_label": "nucleus",
  "gene": "UniProtKB:Q96SF7",
  "gene_symbol": "TBX15",
  "gene_name": "T-box transcription factor TBX15",
  "term_id": "GO:0005634"
}